{
  "term_id": "GO:0007165",
  "gene_name": "Protein FAM83H",
  "gene": "UniProtKB:Q6ZRV2",
  "gene_symbol": "FAM83H",
  "term_label": "signal transduction"
}